{
  "gene": "UniProtKB:Q8IXS8",
  "gene_name": "Hyccin 2",
  "gene_symbol": "HYCC2",
  "term_id": "GO:0046854",
  "term_label": "phosphatidylinositol phosphate biosynthetic process"
}